pericellular basket [GO:1990030] (cellular component) Also known as: peri cellular basket, peri-cellular basket Sources: NIF_Subcellular:sao413722576 Definition: Ramification of basket cell axon surrounding cell bodies, forming the characteristic pericellular baskets from which the cell class derives its name. Relationships: is a type of cellular anatomical structure [GO:0110165]; is part of axon [GO:0030424]